{
  "gene": "UniProtKB:O15432",
  "term_id": "UNKNOWN:0001",
  "gene_name": "Protein SLC31A2",
  "term_label": "Unknown molecular function",
  "gene_symbol": "SLC31A2"
}